{
  "gene": "UniProtKB:Q9Y5Q3",
  "gene_name": "Transcription factor MafB",
  "gene_symbol": "MAFB",
  "term_label": "regulation of transcription by RNA polymerase II",
  "term_id": "GO:0006357"
}